{
  "term_id": "GO:0050829",
  "term_label": "defense response to Gram-negative bacterium",
  "gene": "UniProtKB:P59666",
  "gene_name": "Neutrophil defensin 3",
  "gene_symbol": "DEFA3"
}